{
  "gene": "UniProtKB:P35548",
  "gene_symbol": "MSX2",
  "term_id": "GO:0000977",
  "term_label": "RNA polymerase II transcription regulatory region sequence-specific DNA binding",
  "gene_name": "Homeobox protein MSX-2"
}